nitric-oxide synthase activity [GO:0004517] (molecular function) Relationships: is a type of oxidoreductase activity, acting on paired donors, with incorporation or reduction of molecular oxygen, NAD(P)H as one donor, and incorporation of one atom of oxygen [GO:0016709] Sources: EC:1.14.13.39, RHEA:19897 Also known as: nitric oxide synthase activity, L-arginine,NADPH:oxygen oxidoreductase (nitric-oxide-forming) activity, NADPH-diaphorase activity, NO synthase activity, endothelium-derived relaxation factor-forming enzyme activity, endothelium-derived relaxing factor synthase activity, nitric oxide synthetase activity, nitric-oxide synthetase activity Regulation: regulated by GO:0030235; negatively regulated by nitric-oxide synthase inhibitor activity [GO:0036487]; regulated by regulation of nitric-oxide synthase activity [GO:0050999]; positively regulated by positive regulation of nitric-oxide synthase activity [GO:0051000]; RO_0002212 by negative regulation of nitric-oxide synthase activity [GO:0051001] Definition: Catalysis of the reaction: L-arginine + n NADPH + n H+ + m O2 = citrulline + nitric oxide + n NADP+.